9,13-epoxylabda-14-ene synthase activity [GO:0106239] (molecular function) Relationships: is a type of carbon-oxygen lyase activity, acting on phosphates [GO:0016838] Definition: Catalysis of the reaction:peregrinol diphosphate = (13R)-9,13-epoxylabd-14-ene + diphosphate. References: PMID:24990389 Sources: GOC:emb, RHEA:54512